{
  "gene": "UniProtKB:Q4V326",
  "term_id": "UNKNOWN:0003",
  "gene_name": "G antigen 2E",
  "term_label": "Unknown cellular component",
  "gene_symbol": "GAGE2E"
}